{
  "gene": "UniProtKB:Q8IYA7",
  "term_label": "RNA polymerase II cis-regulatory region sequence-specific DNA binding",
  "gene_symbol": "MKX",
  "gene_name": "Homeobox protein Mohawk",
  "term_id": "GO:0000978"
}